{
  "term_id": "GO:0006357",
  "term_label": "regulation of transcription by RNA polymerase II",
  "gene": "UniProtKB:P21506",
  "gene_name": "Zinc finger protein 10",
  "gene_symbol": "ZNF10"
}